{
  "term_label": "cytoplasm",
  "term_id": "GO:0005737",
  "gene": "UniProtKB:Q8WZ82",
  "gene_name": "Esterase OVCA2",
  "gene_symbol": "OVCA2"
}